{
  "term_label": "plasma membrane",
  "gene_name": "Olfactory receptor 2L13",
  "term_id": "GO:0005886",
  "gene_symbol": "OR2L13",
  "gene": "UniProtKB:Q8N349"
}